{
  "term_label": "somite rostral/caudal axis specification",
  "gene": "UniProtKB:Q9BRJ9",
  "gene_name": "Mesoderm posterior protein 1",
  "gene_symbol": "MESP1",
  "term_id": "GO:0032525"
}